regulation of cap-dependent translational initiation [GO:1903674] (biological process) Sources: GOC:PARL, GOC:TermGenie, GOC:bf, GO_REF:0000058 Definition: Any process that modulates the frequency, rate or extent of cap-dependent translational initiation. Subtypes: negative regulation of cap-dependent translational initiation [GO:1903675], positive regulation of cap-dependent translational initiation [GO:1903676] Relationships: is a type of regulation of cytoplasmic translational initiation [GO:1904688]; regulates GO:0002191